{
  "gene_symbol": "IDS",
  "term_id": "GO:0004423",
  "term_label": "iduronate-2-sulfatase activity",
  "gene_name": "Iduronate 2-sulfatase",
  "gene": "UniProtKB:P22304"
}